dopamine secretion [GO:0014046] (biological process) Relationships: is a type of GO:0015872; is a type of signal release [GO:0023061]; is_a catecholamine secretion [GO:0050432] Subtypes: somato-dendritic dopamine secretion [GO:0099123], axonal dopamine secretion [GO:0099124] Regulation: regulated by GO:0014059; negatively regulated by negative regulation of dopamine secretion [GO:0033602]; positively regulated by positive regulation of dopamine secretion [GO:0033603] Definition: The regulated release of dopamine by a cell. Dopamine is a catecholamine and a precursor of adrenaline and noradrenaline. It acts as a neurotransmitter in the central nervous system but it is also produced peripherally and acts as a hormone. Sources: GOC:ef